negative regulation of mitochondrial fission [GO:0090258] (biological process) Relationships: is a type of negative regulation of organelle organization [GO:0010639]; is a type of GO:0051093; is a type of GO:0090140; negatively regulates mitochondrial fission [GO:0000266] Also known as: negative regulation of mitochondrial division Sources: GOC:sl, GOC:tb Definition: Any process that decreases the rate, frequency or extent of mitochondrial fission. Mitochondrial fission is the division of a mitochondrion within a cell to form two or more separate mitochondrial compartments.